N-terminal peptidyl-serine methylation [GO:0035570] (biological process) Definition: The methylation of the N-terminal serine of proteins. References: PMID:20668449 Relationships: is_a N-terminal protein amino acid methylation [GO:0006480]; is a type of peptidyl-serine modification [GO:0018209] Subtypes: N-terminal peptidyl-serine dimethylation [GO:0035572], N-terminal peptidyl-serine trimethylation [GO:0035573]